{
  "gene": "UniProtKB:P30273",
  "term_id": "GO:0002283",
  "gene_symbol": "FCER1G",
  "term_label": "neutrophil activation involved in immune response",
  "gene_name": "High affinity immunoglobulin epsilon receptor subunit gamma"
}